septin cap [GO:0032159] (cellular component) Relationships: is a type of septin cytoskeleton [GO:0032156]; BFO_0000050 GO:0005856 Subtypes: hyphal septin cap [GO:0032164], germ tube septin cap [GO:0032171] Definition: A faint structure formed of septins found at the leading edge of growth in germ tubes and hyphae in fungal cells growing filamentously. This cap of septins colocalizes with a region of the plasma membrane that is rich in ergosterol. References: PMID:16151244 Sources: GOC:krc